amastigogenesis [GO:0120310] (biological process) Definition: The morphological, biochemical and genetic changes that induce the differentiation of metacyclic parasites into amastigotes in some of the Trypanosomatidae species such as Leishmania parasites and Trypanosoma cruzi. This process occurs inside the cells of the mammalian hosts, particularly in macrophages and other phagocytic cells for Leishmania parasites. Relationships: is a type of development of symbiont in host [GO:0044114] References: PMID:12377273, PMID:13129524, PMID:26752404 Sources: DOI:10.5772/intechopen.84639, GOC:ach, GOC:krc